{
  "term_label": "Unknown cellular component",
  "gene_name": "Putative uncharacterized protein PRO0628",
  "gene_symbol": "PRO0628",
  "gene": "UniProtKB:Q9UI54",
  "term_id": "UNKNOWN:0003"
}